{
  "gene": "UniProtKB:O75431",
  "gene_symbol": "MTX2",
  "gene_name": "Metaxin-2",
  "term_label": "protein insertion into mitochondrial outer membrane",
  "term_id": "GO:0045040"
}